{
  "gene_symbol": "LYZ",
  "term_id": "GO:0003796",
  "term_label": "lysozyme activity",
  "gene": "UniProtKB:P61626",
  "gene_name": "Lysozyme C"
}